{
  "gene_symbol": "HLA-C",
  "gene": "UniProtKB:P10321",
  "gene_name": "HLA class I histocompatibility antigen, C alpha chain",
  "term_id": "GO:0005102",
  "term_label": "signaling receptor binding"
}